{
  "gene_symbol": "WNT5A",
  "gene": "UniProtKB:P41221",
  "gene_name": "Protein Wnt-5a",
  "term_id": "GO:0060070",
  "term_label": "canonical Wnt signaling pathway"
}